{
  "term_label": "Unknown biological process",
  "gene_name": "Keratin-associated protein 23-1",
  "term_id": "UNKNOWN:0002",
  "gene_symbol": "KRTAP23-1",
  "gene": "UniProtKB:A1A580"
}